positive regulation of cilium movement [GO:0003353] (biological process) Definition: Any process that increases the rate, frequency, or extent of cilium movement, the directed, self-propelled movement of a cilium. Sources: GOC:dph Also known as: positive regulation of microtubule-based flagellum movement, positive regulation of flagellar movement, positive regulation of flagellum movement Note: Note that we deem cilium and microtubule-based flagellum to be equivalent. Relationships: is a type of GO:0003352; is a type of positive regulation of cellular process [GO:0048522]; positively regulates GO:0003341 Subtypes: positive regulation of flagellated sperm motility [GO:1902093]